{
  "gene_name": "Zinc finger protein 142",
  "term_label": "regulation of transcription by RNA polymerase II",
  "gene": "UniProtKB:P52746",
  "term_id": "GO:0006357",
  "gene_symbol": "ZNF142"
}